{
  "gene_symbol": "ARTN",
  "term_label": "neuron projection development",
  "gene": "UniProtKB:Q5T4W7",
  "term_id": "GO:0031175",
  "gene_name": "Artemin"
}